{
  "gene_symbol": "MARCHF5",
  "term_label": "mitochondrial outer membrane",
  "term_id": "GO:0005741",
  "gene_name": "E3 ubiquitin-protein ligase MARCHF5",
  "gene": "UniProtKB:Q9NX47"
}